{
  "gene_name": "Exonuclease mut-7 homolog",
  "term_id": "UNKNOWN:0003",
  "gene": "UniProtKB:Q8N9H8",
  "gene_symbol": "EXD3",
  "term_label": "Unknown cellular component"
}